{
  "term_label": "Unknown biological process",
  "gene": "UniProtKB:Q86XT9",
  "gene_name": "Insulin-like growth factor-binding protein 3 receptor",
  "term_id": "UNKNOWN:0002",
  "gene_symbol": "TMEM219"
}